iron-sulfur cluster assembly [GO:0016226] (BP) Subtypes: iron incorporation into metallo-sulfur cluster [GO:0018283], molybdenum incorporation into iron-sulfur cluster [GO:0018291], nickel incorporation into iron-sulfur cluster via tris-L-cysteinyl L-cysteine persulfido L-glutamato L-histidino L-serinyl nickel triiron disulfide trioxide [GO:0018418], [2Fe-2S] cluster assembly [GO:0044571], GO:0044572, GO:0044573, iron-sulfur-molybdenum cofactor assembly [GO:0044593] Relationships: is_a metallo-sulfur cluster assembly [GO:0031163] Also known as: iron-sulphur cluster assembly, iron-sulfur cluster biosynthesis Definition: The incorporation of iron and exogenous sulfur into a metallo-sulfur cluster. Regulation: regulated by regulation of iron-sulfur cluster assembly [GO:1903329]; negatively regulated by negative regulation of iron-sulfur cluster assembly [GO:1903330]; positively regulated by positive regulation of iron-sulfur cluster assembly [GO:1903331] Sources: GOC:jl, GOC:mah, GOC:pde, GOC:vw